L-galactonate catabolic process [GO:0034195] (biological process) Also known as: L-galactonate breakdown, L-galactonate catabolism, L-galactonate degradation Definition: The chemical reactions and pathways resulting in the breakdown of L-galactonate, the anion of L-galactonic acid. Relationships: is a type of GO:0016052; is a type of GO:0019584 Sources: GOC:ai, GOC:mah